alkanesulfonate monooxygenase complex [GO:1990201] (cellular component) Relationships: is a type of GO:1990204; is part of cytosol [GO:0005829] References: PMID:10480865, PMID:16997955 Sources: GOC:bhm Also known as: SsuD complex Definition: A protein complex capable of alkanesulfonate monooxygenase activity. Involved in the utilization of alkanesulfonates as sulfur sources under conditions of sulfate or cysteine starvation, catalyzing the conversion of alkanesulfonates into aldehydes and sulfite. In E.coli the complex consists of a SsuD tetramer.